ecdysteroid catabolic process [GO:0046344] (biological process) Subtypes: ecdysone catabolic process [GO:0006708] Also known as: ecdysteroid breakdown, ecdysteroid catabolism, ecdysteroid degradation Definition: The chemical reactions and pathways resulting in the breakdown of ecdysteroids, a group of polyhydroxylated ketosteroids which initiate post-embryonic development. Sources: GOC:ai Relationships: is a type of GO:0006706; is a type of GO:0042182; is a type of hormone catabolic process [GO:0042447]; is a type of ecdysteroid metabolic process [GO:0045455]